{
  "term_label": "extracellular space",
  "term_id": "GO:0005615",
  "gene_name": "Beta-nerve growth factor",
  "gene": "UniProtKB:P01138",
  "gene_symbol": "NGF"
}